{
  "gene_name": "Synaptotagmin-9",
  "gene": "UniProtKB:Q86SS6",
  "gene_symbol": "SYT9",
  "term_id": "GO:0005544",
  "term_label": "calcium-dependent phospholipid binding"
}